muscle structure development [GO:0061061] (biological process) Relationships: is a type of GO:0048856 Sources: GOC:dph Subtypes: GO:0007517, GO:0007525 Definition: The progression of a muscle structure over time, from its formation to its mature state. Muscle structures are contractile cells, tissues or organs that are found in multicellular organisms.